L-erythro-3-methylmalyl-CoA lyase activity [GO:0043959] (molecular function) Also known as: HpcH/HpaI aldolase Sources: RHEA:38259 Relationships: is a type of GO:0016833 Definition: Catalysis of the reaction: (2R,3S)-beta-methylmalyl-CoA = glyoxylate + propanoyl-CoA.